{
  "term_label": "Unknown biological process",
  "gene_symbol": "EIF4H",
  "term_id": "UNKNOWN:0002",
  "gene_name": "Eukaryotic translation initiation factor 4H",
  "gene": "UniProtKB:Q15056"
}